flap-structured DNA binding [GO:0070336] (molecular function) Definition: Binding to a flap structure in DNA. A DNA flap structure is one in which a single-stranded length of DNA or RNA protrudes from a double-stranded DNA molecule. References: PMID:15189154 Sources: GOC:mah Relationships: is a type of DNA binding [GO:0003677] Subtypes: 3'-flap-structured DNA binding [GO:0070337], GO:0070338